lumenal side of cis-Golgi network membrane [GO:0140178] (CC) Relationships: is a type of lumenal side of membrane [GO:0098576]; is part of GO:0033106 Definition: The membrane leaflet of the cis-Golgi network directly contacts the Golgi lumen and may be involved in glycosylation, cargo sorting, or interactions with resident Golgi proteins. References: PMID:1747103, PMID:29802621, PMID:34080016